{
  "gene": "UniProtKB:Q6IPU0",
  "term_label": "nucleus",
  "gene_symbol": "CENPP",
  "term_id": "GO:0005634",
  "gene_name": "Centromere protein P"
}